{
  "gene": "UniProtKB:A0FGR8",
  "gene_symbol": "ESYT2",
  "gene_name": "Extended synaptotagmin-2",
  "term_label": "phosphatidylinositol binding",
  "term_id": "GO:0035091"
}